positive regulation of the force of heart contraction by circulating norepinephrine [GO:0003109] (biological process) Also known as: increased force of heart contraction by circulating norepinephrine, increased force of heart contraction by circulating noradrenaline Definition: The process in which the secretion of norepinephrine into the bloodstream modulates the force of heart muscle contraction. Sources: GOC:mtg_cardio Relationships: is a type of positive regulation of the force of heart contraction by norepinephrine [GO:0003061]